{
  "term_label": "Unknown molecular function",
  "gene_symbol": "CROCC2",
  "gene_name": "Ciliary rootlet coiled-coil protein 2",
  "term_id": "UNKNOWN:0001",
  "gene": "UniProtKB:H7BZ55"
}